determination of heart left/right asymmetry [GO:0061371] (biological process) Also known as: determination of cardiac left/right asymmetry Sources: GOC:dph, GOC:mtg_heart Relationships: is a type of determination of left/right symmetry [GO:0007368]; BFO_0000050 heart development [GO:0007507] Definition: Determination of the asymmetric location of the heart with respect to the left and right halves of the organism.